10-hydroxygeraniol oxidoreductase activity [GO:0102967] (molecular function) Relationships: is a type of oxidoreductase activity, acting on the CH-OH group of donors, NAD or NADP as acceptor [GO:0016616] Sources: GOC:pz, RHEA:32607 Definition: Catalysis of the reaction: (6E)-8-hydroxygeraniol + NADP = (6E)-8-hydroxygeranial + NADPH + H+.